{
  "gene": "UniProtKB:O43581",
  "term_label": "synaptic vesicle",
  "term_id": "GO:0008021",
  "gene_symbol": "SYT7",
  "gene_name": "Synaptotagmin-7"
}